{
  "gene": "UniProtKB:Q96PC5",
  "term_id": "GO:0009306",
  "gene_name": "Melanoma inhibitory activity protein 2",
  "term_label": "protein secretion",
  "gene_symbol": "MIA2"
}